{
  "term_label": "ubiquitin protein ligase activity",
  "gene_symbol": "RNF11",
  "term_id": "GO:0061630",
  "gene": "UniProtKB:Q9Y3C5",
  "gene_name": "RING finger protein 11"
}